connexin complex [GO:0005922] (cellular component) Relationships: is a type of plasma membrane protein complex [GO:0098797]; is part of gap junction [GO:0005921] References: PMID:11146276 Also known as: connexon, connexon complex Definition: An assembly of six molecules of connexin, made in the Golgi apparatus and subsequently transported to the plasma membrane, where docking of two connexons on apposed plasma membranes across the extracellular space forms a gap junction.